{
  "term_id": "GO:0005737",
  "gene_symbol": "PRAMEF6",
  "term_label": "cytoplasm",
  "gene_name": "PRAME family member 6",
  "gene": "UniProtKB:Q5VXH4"
}